contractile vacuole [GO:0000331] (cellular component) Definition: A specialized vacuole of eukaryotic cells, especially Protozoa, that fills with water from the cytoplasm and then discharges this externally by the opening of contractile vacuole pores. One of its functions is osmoregulatory. References: PMID:10503189, PMID:23890380 Sources: GOC:jl Relationships: is a type of GO:0005773; is a type of GO:0031410; is part of contractile vacuole complex [GO:0062159] Also known as: central bladder, central vacuole